{
  "term_id": "GO:0004984",
  "gene_name": "Olfactory receptor 2H2",
  "gene_symbol": "OR2H2",
  "term_label": "olfactory receptor activity",
  "gene": "UniProtKB:O95918"
}